{
  "gene_symbol": "PRKY",
  "term_id": "GO:0005952",
  "gene_name": "Putative serine_threonine-protein kinase PRKY",
  "term_label": "cAMP-dependent protein kinase complex",
  "gene": "UniProtKB:O43930"
}